{
  "term_label": "regulation of microtubule polymerization or depolymerization",
  "term_id": "GO:0031110",
  "gene_name": "GAS2-like protein 1",
  "gene_symbol": "GAS2L1",
  "gene": "UniProtKB:Q99501"
}